protein secretion by the type VI secretion system [GO:0033103] (biological process) Relationships: is a type of GO:0009306; is a type of protein transmembrane transport [GO:0071806] Also known as: protein secretion by the T6SS, protein secretion by the type VI protein secretion system, type VI protein secretion system Note: Note that this term represents an activity and not a cellular structure. Consider also annotating to the cellular component term 'type VI protein secretion system complex ; GO:0033104'. Definition: The process in which proteins are transferred into the extracellular milieu or directly into host cells by the type VI secretion system. Proteins secreted by this system do not require an N-terminal signal sequence. References: PMID:16432199, PMID:16763151 Sources: GOC:mlg